{
  "gene_symbol": "C2CD4A",
  "term_label": "Unknown cellular component",
  "term_id": "UNKNOWN:0003",
  "gene_name": "C2 calcium-dependent domain-containing protein 4A",
  "gene": "UniProtKB:Q8NCU7"
}